{
  "term_id": "GO:1902600",
  "gene_name": "Proton channel OTOP3",
  "gene_symbol": "OTOP3",
  "term_label": "proton transmembrane transport",
  "gene": "UniProtKB:Q7RTS5"
}